polyol transmembrane transporter activity [GO:0015166] (molecular function) Sources: ISBN:0198506732 Also known as: sugar/polyol channel activity Relationships: is a type of transmembrane transporter activity [GO:0022857]; is part of polyol transmembrane transport [GO:0015791] Subtypes: myo-inositol transmembrane transporter activity [GO:0005365], GO:0015167, GO:0015168, mannitol transmembrane transporter activity [GO:0015575], sorbitol transmembrane transporter activity [GO:0015576], GO:0015577, chloramphenicol transmembrane transporter activity [GO:0042896], glucosylglycerol transmembrane transporter activity [GO:0051474] Definition: Enables the transfer of a polyol from one side of a membrane to the other. A polyol is any polyhydric alcohol.